{
  "gene_name": "Homeobox protein HMX2",
  "gene_symbol": "HMX2",
  "term_id": "GO:0006357",
  "gene": "UniProtKB:A2RU54",
  "term_label": "regulation of transcription by RNA polymerase II"
}